{
  "term_label": "Unknown cellular component",
  "gene_name": "Tetratricopeptide repeat protein 5",
  "gene": "UniProtKB:Q8N0Z6",
  "term_id": "UNKNOWN:0003",
  "gene_symbol": "TTC5"
}